{
  "term_id": "GO:0004527",
  "gene_symbol": "REXO4",
  "gene": "UniProtKB:Q9GZR2",
  "gene_name": "RNA exonuclease 4",
  "term_label": "exonuclease activity"
}